{
  "term_id": "GO:0030527",
  "gene_name": "Histone H2A",
  "term_label": "structural constituent of chromatin",
  "gene": "UniProtKB:A0A8Q3WKH5",
  "gene_symbol": "H2AL1Q"
}